{
  "gene_symbol": "RNF138",
  "term_id": "GO:0000724",
  "term_label": "double-strand break repair via homologous recombination",
  "gene": "UniProtKB:Q8WVD3",
  "gene_name": "E3 ubiquitin-protein ligase RNF138"
}